chemorepulsion involved in embryonic olfactory bulb interneuron precursor migration [GO:0021834] (biological process) Also known as: negative chemotaxis involved in embryonic olfactory bulb interneuron precursor migration References: PMID:12626695 Sources: GOC:cls, GOC:dgh, GOC:dph, GOC:jid, GO_REF:0000021 Definition: The creation and reception of signals that guide olfactory bulb interneuron precursors down concentration gradients towards the olfactory bulb. Relationships: is a type of GO:0050919; is part of embryonic olfactory bulb interneuron precursor migration [GO:0021831]